inositol-1,3,4,6-tetrakisphosphate 2-kinase activity [GO:0102731] (molecular function) Relationships: is a type of inositol tetrakisphosphate kinase activity [GO:0051765] References: PMID:16107538 Sources: MetaCyc:RXN-7185 Definition: Catalysis of the reaction: 1D-myo-inositol 1,3,4,6-tetrakisphosphate + ATP = 1D-myo-inositol 1,2,3,4,6-pentakisphosphate + ADP + H+. Also known as: D-myo-inositol (1,3,4,6)-tetrakisphosphate 2-kinase activity